hair cycle process [GO:0022405] (biological process) Sources: GOC:isa_complete Definition: A multicellular organismal process involved in the cyclical phases of growth (anagen), regression (catagen), quiescence (telogen), and shedding (exogen) in the life of a hair; one of the collection or mass of filaments growing from the skin of an animal, and forming a covering for a part of the head or for any part or the whole of the body. Relationships: is a type of molting cycle process [GO:0022404]; is part of hair cycle [GO:0042633] Subtypes: hair follicle development [GO:0001942], GO:0031069, GO:0048820